{
  "gene_name": "Oligodendrocyte transcription factor 1",
  "term_label": "DNA-binding transcription factor activity, RNA polymerase II-specific",
  "term_id": "GO:0000981",
  "gene": "UniProtKB:Q8TAK6",
  "gene_symbol": "OLIG1"
}